{
  "gene_name": "Ras-related GTP-binding protein A",
  "gene_symbol": "RRAGA",
  "gene": "UniProtKB:Q7L523",
  "term_id": "GO:0005764",
  "term_label": "lysosome"
}